{
  "term_id": "GO:0035091",
  "gene_name": "Sorting nexin-31",
  "term_label": "phosphatidylinositol binding",
  "gene": "UniProtKB:Q8N9S9",
  "gene_symbol": "SNX31"
}